{
  "gene_symbol": "TBX20",
  "gene": "UniProtKB:Q9UMR3",
  "gene_name": "T-box transcription factor TBX20",
  "term_label": "nucleus",
  "term_id": "GO:0005634"
}